{
  "gene_symbol": "SOX17",
  "gene_name": "Transcription factor SOX-17",
  "term_label": "DNA-binding transcription activator activity, RNA polymerase II-specific",
  "term_id": "GO:0001228",
  "gene": "UniProtKB:Q9H6I2"
}